negative regulation of diorcinol biosynthetic process [GO:1900656] (biological process) Relationships: is a type of negative regulation of secondary metabolite biosynthetic process [GO:1900377]; is a type of regulation of diorcinol biosynthetic process [GO:1900655]; negatively regulates diorcinol biosynthetic process [GO:1900572] Definition: Any process that stops, prevents or reduces the frequency, rate or extent of diorcinol biosynthetic process. Sources: GOC:TermGenie, GOC:di Also known as: down regulation of diorcinol anabolism, down regulation of diorcinol biosynthesis, down regulation of diorcinol biosynthetic process, down regulation of diorcinol formation, down regulation of diorcinol synthesis, down-regulation of diorcinol anabolism, down-regulation of diorcinol biosynthesis, down-regulation of diorcinol biosynthetic process, down-regulation of diorcinol formation, down-regulation of diorcinol synthesis, downregulation of diorcinol anabolism, downregulation of diorcinol biosynthesis, downregulation of diorcinol biosynthetic process, downregulation of diorcinol formation, downregulation of diorcinol synthesis, inhibition of diorcinol anabolism, inhibition of diorcinol biosynthesis, inhibition of diorcinol formation, inhibition of diorcinol synthesis, negative regulation of diorcinol anabolism, negative regulation of diorcinol biosynthesis, negative regulation of diorcinol formation, negative regulation of diorcinol synthesis, inhibition of diorcinol biosynthetic process